{
  "term_label": "3',5'-cyclic-AMP phosphodiesterase activity",
  "gene": "UniProtKB:Q07343",
  "term_id": "GO:0004115",
  "gene_name": "cAMP-specific 3',5'-cyclic phosphodiesterase 4B",
  "gene_symbol": "PDE4B"
}